{
  "term_label": "cuprous ion binding",
  "gene_name": "Gamma-synuclein",
  "term_id": "GO:1903136",
  "gene": "UniProtKB:O76070",
  "gene_symbol": "SNCG"
}